{
  "gene": "UniProtKB:Q9NP62",
  "gene_name": "Chorion-specific transcription factor GCMa",
  "gene_symbol": "GCM1",
  "term_id": "GO:0042063",
  "term_label": "gliogenesis"
}